{
  "term_label": "regulation of transcription by RNA polymerase II",
  "gene_symbol": "PAX5",
  "term_id": "GO:0006357",
  "gene_name": "Paired box protein Pax-5",
  "gene": "UniProtKB:Q02548"
}